{
  "gene_symbol": "TOMM70",
  "term_id": "GO:0008320",
  "gene": "UniProtKB:O94826",
  "gene_name": "Mitochondrial import receptor subunit TOM70",
  "term_label": "protein transmembrane transporter activity"
}